{
  "gene_name": "Menin",
  "term_label": "regulation of transcription by RNA polymerase II",
  "gene": "UniProtKB:O00255",
  "gene_symbol": "MEN1",
  "term_id": "GO:0006357"
}